{
  "gene_name": "Bifunctional UDP-N-acetylglucosamine 2-epimerase_N-acetylmannosamine kinase",
  "gene": "UniProtKB:Q9Y223",
  "term_label": "Unknown cellular component",
  "term_id": "UNKNOWN:0003",
  "gene_symbol": "GNE"
}